{
  "term_id": "GO:0006413",
  "gene_symbol": "EIF4G1",
  "gene_name": "Eukaryotic translation initiation factor 4 gamma 1",
  "gene": "UniProtKB:Q04637",
  "term_label": "translational initiation"
}